myelination [GO:0042552] (biological process) Relationships: is a type of axon ensheathment [GO:0008366] Also known as: myelinogenesis Sources: GOC:dgh, GOC:mah Regulation: regulated by GO:0031641; negatively regulated by negative regulation of myelination [GO:0031642]; positively regulated by positive regulation of myelination [GO:0031643] Subtypes: central nervous system myelination [GO:0022010], myelination in peripheral nervous system [GO:0022011], myelination of lateral line nerve axons [GO:0048897] Definition: The process in which myelin sheaths are formed and maintained around neurons. Oligodendrocytes in the brain and spinal cord and Schwann cells in the peripheral nervous system wrap axons with compact layers of their plasma membrane. Adjacent myelin segments are separated by a non-myelinated stretch of axon called a node of Ranvier.